{
  "gene": "UniProtKB:Q96MI9",
  "term_id": "GO:0015630",
  "gene_name": "Cytosolic carboxypeptidase 4",
  "gene_symbol": "AGBL1",
  "term_label": "microtubule cytoskeleton"
}